{
  "gene": "UniProtKB:Q15642",
  "gene_name": "Cdc42-interacting protein 4",
  "gene_symbol": "TRIP10",
  "term_id": "UNKNOWN:0002",
  "term_label": "Unknown biological process"
}